thioredoxin-dependent peroxiredoxin activity [GO:0140824] (MF) Relationships: is a type of peroxiredoxin activity [GO:0051920] Subtypes: GO:0008379 Definition: Catalysis of the reaction: [thioredoxin]-dithiol + a hydroperoxide = [thioredoxin]-disulfide + an alcohol + H2O. References: PMID:12707274, PMID:19820102 Sources: RHEA:62620